{
  "term_label": "Tie signaling pathway",
  "gene": "UniProtKB:O15123",
  "term_id": "GO:0048014",
  "gene_symbol": "ANGPT2",
  "gene_name": "Angiopoietin-2"
}